{
  "gene_name": "Heat shock protein HSP 90-alpha A2",
  "term_id": "GO:0050821",
  "gene": "UniProtKB:Q14568",
  "gene_symbol": "HSP90AA2P",
  "term_label": "protein stabilization"
}